{
  "gene_name": "Putative protein FAM90A22",
  "term_label": "Unknown biological process",
  "gene_symbol": "FAM90A22",
  "term_id": "UNKNOWN:0002",
  "gene": "UniProtKB:A8MWA6"
}